{
  "term_id": "GO:0007265",
  "gene_symbol": "RGL3",
  "gene_name": "Ral guanine nucleotide dissociation stimulator-like 3",
  "gene": "UniProtKB:Q3MIN7",
  "term_label": "Ras protein signal transduction"
}